lipid III floppase activity [GO:0015161] (molecular function) Also known as: capsule polysaccharide transporter activity, undecaprenol-pyrophosphate O-antigen flippase activity, capsular polysaccharide transmembrane transporter activity Relationships: is a type of floppase activity [GO:0140328]; is part of capsular polysaccharide transport [GO:0015776] Definition: Enables the transbilayer of capsular-polysaccharides (Und-PP-GlcNAc-ManNAcA-Fuc4NAc (lipid III)) from the inner to the outer leaflet of the cytoplasmic membrane during the assembly of ECA. Capsular polysaccharides make up the capsule, a protective structure surrounding some species of bacteria and fungi. References: PMID:12621029, PMID:16816184 Sources: GOC:ai, GOC:mtg_transport